stereocilium shaft [GO:0120043] (cellular component) Definition: The shaft comprises the majority of the length of the stereocilium. This region is notable for the extreme stability of actin filaments, which are highly crosslinked into a parallel bundle. Relationships: is a type of cellular anatomical structure [GO:0110165]; is part of stereocilium [GO:0032420] References: PMID:20170899 Sources: GOC:krc